{
  "gene": "UniProtKB:Q5VT66",
  "term_label": "molybdopterin cofactor binding",
  "term_id": "GO:0043546",
  "gene_symbol": "MTARC1",
  "gene_name": "Mitochondrial amidoxime-reducing component 1"
}